{
  "gene": "UniProtKB:Q9H1K4",
  "term_id": "GO:0005313",
  "gene_name": "Mitochondrial glutamate carrier 2",
  "gene_symbol": "SLC25A18",
  "term_label": "L-glutamate transmembrane transporter activity"
}